metanephric glomerulus development [GO:0072224] (biological process) Regulation: regulated by regulation of metanephric glomerulus development [GO:0072298]; negatively regulated by negative regulation of metanephric glomerulus development [GO:0072299]; positively regulated by positive regulation of metanephric glomerulus development [GO:0072300] Sources: GOC:mah Relationships: is a type of glomerulus development [GO:0032835]; is part of metanephric nephron development [GO:0072210] Also known as: metanephric glomerular development Definition: The progression of the metanephric glomerulus over time from its initial formation until its mature state. The metanephric glomerulus is a capillary tuft which forms a close network with the visceral epithelium (podocytes) and the mesangium to form the filtration barrier and is surrounded by Bowman's capsule in nephrons of the mature vertebrate kidney, or metanephros.